{
  "gene_name": "Prolactin",
  "term_id": "GO:0005179",
  "gene_symbol": "PRL",
  "gene": "UniProtKB:P01236",
  "term_label": "hormone activity"
}